{
  "gene": "UniProtKB:Q9BTA9",
  "gene_symbol": "WAC",
  "term_id": "GO:0005634",
  "gene_name": "WW domain-containing adapter protein with coiled-coil",
  "term_label": "nucleus"
}